multivesicular body lumen [GO:0097486] (cellular component) Definition: The volume enclosed by the outermost membrane of a multivesicular body. References: PMID:21183070 Sources: GOC:pde Relationships: is a type of late endosome lumen [GO:0031906]; is part of multivesicular body [GO:0005771]